translation at postsynapse [GO:0140242] (biological process) Note: Note that this term was created for the SynGO project, and will be obsoleted when the SynGO annotations are made in Noctua. Definition: Translation that occurs at the postsynapse. References: PMID:20427644 Relationships: is a type of GO:0140241; occurs in GO:0098794